sinus venosus morphogenesis [GO:0003236] (biological process) Definition: The process in which the sinus venosus is generated and organized. The sinus venosus is a heart chamber attached to the atrium on the venous side of the embryonic heart. Sources: GOC:mtg_heart Relationships: is a type of cardiac chamber morphogenesis [GO:0003206]; is part of sinus venosus development [GO:0003235]